positive regulation of phytol biosynthetic process [GO:1904964] (biological process) References: PMID:24275650 Sources: GOC:TermGenie, GO_REF:0000058 Definition: Any process that activates or increases the frequency, rate or extent of phytol biosynthetic process. Also known as: positive regulation of phytol anabolism, positive regulation of phytol biosynthesis, positive regulation of phytol formation, positive regulation of phytol synthesis, up regulation of phytol anabolism, up regulation of phytol biosynthesis, up regulation of phytol biosynthetic process, up regulation of phytol formation, up regulation of phytol synthesis, up-regulation of phytol anabolism, up-regulation of phytol biosynthesis, up-regulation of phytol biosynthetic process, up-regulation of phytol formation, up-regulation of phytol synthesis, upregulation of phytol anabolism, upregulation of phytol biosynthesis, upregulation of phytol biosynthetic process, upregulation of phytol formation, upregulation of phytol synthesis, activation of phytol anabolism, activation of phytol biosynthesis, activation of phytol biosynthetic process, activation of phytol formation, activation of phytol synthesis Relationships: is a type of positive regulation of lipid biosynthetic process [GO:0046889]; is a type of positive regulation of alcohol biosynthetic process [GO:1902932]; is_a regulation of phytol biosynthetic process [GO:1904963]; positively regulates GO:0033520